{
  "term_id": "UNKNOWN:0002",
  "term_label": "Unknown biological process",
  "gene_symbol": "TAGAP",
  "gene": "UniProtKB:Q8N103",
  "gene_name": "T-cell activation Rho GTPase-activating protein"
}